dorsal/ventral lineage restriction, imaginal disc [GO:0007451] (biological process) Also known as: dorsal-ventral lineage restriction, imaginal disc, dorsoventral lineage restriction, imaginal disc References: PMID:10625531, PMID:9374402 Sources: GOC:bf Definition: Formation and/or maintenance of a lineage boundary between dorsal and ventral compartments that cells cannot cross, thus separating the populations of cells in each compartment. Relationships: is_a imaginal disc lineage restriction [GO:0035161]; is part of dorsal/ventral pattern formation, imaginal disc [GO:0007450]